cellular response to nitroglycerin [GO:1904843] (biological process) References: PMID:25626975 Sources: GOC:TermGenie, GO_REF:0000071 Definition: Any process that results in a change in state or activity of a cell (in terms of movement, secretion, enzyme production, gene expression, etc.) as a result of a nitroglycerin stimulus. Also known as: cellular response to nitroglycerine, cellular response to nitroglycerol, cellular response to trinitroglycerin, cellular response to trinitroglycerol Relationships: is a type of cellular response to nitrogen compound [GO:1901699]; is a type of GO:1901701; is a type of response to nitroglycerin [GO:1904842]